structural constituent of cuticle [GO:0042302] (molecular function) Relationships: is a type of GO:0005198 Definition: The action of a molecule that contributes to the structural integrity of a cuticle. Sources: GOC:jl Subtypes: GO:0005214, structural constituent of collagen and cuticulin-based cuticle [GO:0042329]